{
  "gene": "UniProtKB:P35030",
  "term_label": "proteolysis",
  "gene_name": "Trypsin-3",
  "term_id": "GO:0006508",
  "gene_symbol": "PRSS3"
}